{
  "term_label": "cytoplasm",
  "gene_name": "Serine_Arginine-related protein 53",
  "term_id": "GO:0005737",
  "gene": "UniProtKB:Q96IZ7",
  "gene_symbol": "RSRC1"
}